{
  "gene": "UniProtKB:Q8N4F7",
  "term_label": "ERAD pathway",
  "gene_symbol": "RNF175",
  "gene_name": "RING finger protein 175",
  "term_id": "GO:0036503"
}